positive regulation of macrophage cytokine production [GO:0060907] (biological process) Definition: Any process that increases the rate, frequency or extent of macrophage cytokine production. Macrophage cytokine production is the appearance of a chemokine due to biosynthesis or secretion following a cellular stimulus, resulting in an increase in its intracellular or extracellular levels. Sources: GOC:dph, GOC:tb Relationships: is a type of regulation of macrophage cytokine production [GO:0010935]; is a type of GO:0061081; positively regulates macrophage cytokine production [GO:0010934]